{
  "gene_name": "Mothers against decapentaplegic homolog 7",
  "gene": "UniProtKB:O15105",
  "gene_symbol": "SMAD7",
  "term_label": "regulation of transcription by RNA polymerase II",
  "term_id": "GO:0006357"
}